negative regulation of leukocyte degranulation [GO:0043301] (biological process) Sources: GOC:add, ISBN:0781735149 Relationships: is a type of negative regulation of immune effector process [GO:0002698]; is a type of regulation of leukocyte degranulation [GO:0043300]; is_a negative regulation of regulated secretory pathway [GO:1903306]; negatively regulates leukocyte degranulation [GO:0043299] Definition: Any process that stops, prevents, or reduces the rate of leukocyte degranulation. Subtypes: negative regulation of mast cell degranulation [GO:0043305], negative regulation of eosinophil degranulation [GO:0043310], negative regulation of neutrophil degranulation [GO:0043314], GO:0043318, negative regulation of natural killer cell degranulation [GO:0043322], negative regulation of basophil degranulation [GO:1903582] Also known as: down regulation of leukocyte degranulation, down-regulation of leukocyte degranulation, downregulation of leukocyte degranulation, negative regulation of immune cell degranulation, negative regulation of leucocyte degranulation, inhibition of leukocyte degranulation